{
  "term_label": "calmodulin binding",
  "term_id": "GO:0005516",
  "gene_name": "Ras GTPase-activating-like protein IQGAP1",
  "gene_symbol": "IQGAP1",
  "gene": "UniProtKB:P46940"
}